positive regulation of prostaglandin catabolic process [GO:1905830] (biological process) Also known as: positive regulation of prostaglandin breakdown, positive regulation of prostaglandin catabolism, positive regulation of prostaglandin degradation, up regulation of prostaglandin breakdown, up regulation of prostaglandin catabolic process, up regulation of prostaglandin catabolism, up regulation of prostaglandin degradation, up-regulation of prostaglandin breakdown, up-regulation of prostaglandin catabolic process, up-regulation of prostaglandin catabolism, up-regulation of prostaglandin degradation, upregulation of prostaglandin breakdown, upregulation of prostaglandin catabolic process, upregulation of prostaglandin catabolism, upregulation of prostaglandin degradation, activation of prostaglandin breakdown, activation of prostaglandin catabolic process, activation of prostaglandin catabolism, activation of prostaglandin degradation References: PMID:12432938 Sources: GOC:TermGenie, GO_REF:0000058 Definition: Any process that activates or increases the frequency, rate or extent of prostaglandin catabolic process. Relationships: is a type of positive regulation of lipid catabolic process [GO:0050996]; is a type of regulation of prostaglandin catabolic process [GO:1905828]; positively regulates prostaglandin catabolic process [GO:1905344]